{
  "term_id": "GO:0043066",
  "gene_name": "Epidermal growth factor receptor",
  "gene_symbol": "EGFR",
  "term_label": "negative regulation of apoptotic process",
  "gene": "UniProtKB:P00533"
}